seryl-selenocysteinyl-tRNA kinase activity [GO:0098620] (molecular function) Relationships: is a type of phosphotransferase activity, alcohol group as acceptor [GO:0016773]; is a type of catalytic activity, acting on a tRNA [GO:0140101] Definition: Catalysis of the reaction: Ser-tRNA(Sec) + ATP = Sep-tRNA(Sec) + ADP. References: PMID:15317934